{
  "term_id": "GO:0005096",
  "gene": "UniProtKB:Q08116",
  "gene_name": "Regulator of G-protein signaling 1",
  "gene_symbol": "RGS1",
  "term_label": "GTPase activator activity"
}